positive regulation of glutamate uptake involved in transmission of nerve impulse [GO:0051951] (biological process) Definition: Any process that activates, maintains or increases the frequency, rate or extent of the directed movement of L-glutamate into a neuron or glial cell. Also known as: positive regulation of glutamate reuptake, positive regulation of glutamate uptake involved in conduction of nerve impulse, up regulation of glutamate uptake during transmission of nerve impulse, up-regulation of glutamate uptake during transmission of nerve impulse, upregulation of glutamate uptake during transmission of nerve impulse, activation of glutamate uptake during transmission of nerve impulse, stimulation of glutamate uptake during transmission of nerve impulse, positive regulation of glutamate uptake during transmission of nerve impulse Sources: GOC:ai Relationships: is a type of positive regulation of L-glutamate import across plasma membrane [GO:0002038]; is a type of positive regulation of amino acid uptake involved in synaptic transmission [GO:0051943]; is_a regulation of glutamate uptake involved in transmission of nerve impulse [GO:0051946]; positively regulates GO:0051935